{
  "gene_name": "RNA polymerase II subunit A C-terminal domain phosphatase SSU72 like protein 4",
  "term_id": "GO:0008420",
  "gene_symbol": "SSU72L4",
  "term_label": "RNA polymerase II CTD heptapeptide repeat phosphatase activity",
  "gene": "UniProtKB:A0A1W2PQC6"
}